{
  "gene_name": "Transmembrane 4 L6 family member 18",
  "gene": "UniProtKB:Q96CE8",
  "term_id": "GO:0016020",
  "gene_symbol": "TM4SF18",
  "term_label": "membrane"
}